{
  "gene_name": "Olfactory receptor 4X2",
  "term_id": "UNKNOWN:0002",
  "term_label": "Unknown biological process",
  "gene_symbol": "OR4X2",
  "gene": "UniProtKB:Q8NGF9"
}